epothilone biosynthetic process [GO:0050814] (biological process) Definition: The chemical reactions and pathways resulting in the formation of epothilone, a drug obtained from the myxobacteria Sporangium cellulosum that interferes with cell division. Some epothilones are being studied as treatments for cancer. Sources: GOC:ai Also known as: epothilone anabolism, epothilone biosynthesis, epothilone formation, epothilone synthesis Relationships: is a type of macrolide biosynthetic process [GO:0033068]; is a type of ketone biosynthetic process [GO:0042181]; is a type of sulfur compound biosynthetic process [GO:0044272]